{
  "gene_symbol": "TMEM177",
  "term_label": "Unknown biological process",
  "gene_name": "Transmembrane protein 177",
  "term_id": "UNKNOWN:0002",
  "gene": "UniProtKB:Q53S58"
}